{
  "gene_symbol": "MTPN",
  "gene_name": "Myotrophin",
  "term_label": "nucleus",
  "gene": "UniProtKB:P58546",
  "term_id": "GO:0005634"
}